{
  "term_label": "plasma membrane",
  "term_id": "GO:0005886",
  "gene_symbol": "ANO8",
  "gene": "UniProtKB:Q9HCE9",
  "gene_name": "Anoctamin-8"
}